{
  "gene_symbol": "DNAJC30",
  "term_id": "UNKNOWN:0001",
  "gene": "UniProtKB:Q96LL9",
  "term_label": "Unknown molecular function",
  "gene_name": "DnaJ homolog subfamily C member 30, mitochondrial"
}